{
  "gene_symbol": "CD300H",
  "term_id": "GO:0004888",
  "term_label": "transmembrane signaling receptor activity",
  "gene_name": "Protein CD300H",
  "gene": "UniProtKB:A0A0K2S4Q6"
}